{
  "gene_name": "Methyl-CpG-binding domain protein 4",
  "term_label": "nucleus",
  "term_id": "GO:0005634",
  "gene": "UniProtKB:O95243",
  "gene_symbol": "MBD4"
}